{
  "term_id": "GO:0090364",
  "gene": "UniProtKB:Q8WVY7",
  "term_label": "regulation of proteasome assembly",
  "gene_symbol": "UBLCP1",
  "gene_name": "Ubiquitin-like domain-containing CTD phosphatase 1"
}